{
  "term_id": "UNKNOWN:0002",
  "gene_name": "Zona pellucida-like domain-containing protein 1",
  "gene_symbol": "ZPLD1",
  "term_label": "Unknown biological process",
  "gene": "UniProtKB:Q8TCW7"
}